{
  "term_id": "GO:0042910",
  "gene_symbol": "ABCB1",
  "term_label": "xenobiotic transmembrane transporter activity",
  "gene_name": "ATP-dependent translocase ABCB1",
  "gene": "UniProtKB:P08183"
}